{
  "gene_name": "Septin-4",
  "gene_symbol": "SEPTIN4",
  "term_id": "GO:0031105",
  "gene": "UniProtKB:O43236",
  "term_label": "septin complex"
}